positive regulation of camalexin biosynthetic process [GO:1901183] (biological process) Also known as: activation of camalexin anabolism, activation of camalexin biosynthesis, activation of camalexin formation, activation of camalexin synthesis, positive regulation of camalexin anabolism, positive regulation of camalexin biosynthesis, positive regulation of camalexin formation, positive regulation of camalexin synthesis, up regulation of camalexin anabolism, up regulation of camalexin biosynthesis, up regulation of camalexin biosynthetic process, up regulation of camalexin formation, up regulation of camalexin synthesis, up-regulation of camalexin anabolism, up-regulation of camalexin biosynthesis, up-regulation of camalexin biosynthetic process, up-regulation of camalexin formation, up-regulation of camalexin synthesis, upregulation of camalexin anabolism, upregulation of camalexin biosynthesis, upregulation of camalexin biosynthetic process, upregulation of camalexin formation, upregulation of camalexin synthesis, activation of camalexin biosynthetic process Relationships: is a type of regulation of sulfur metabolic process [GO:0042762]; is a type of positive regulation of phytoalexin biosynthetic process [GO:0052322]; positively regulates camalexin biosynthetic process [GO:0010120] Sources: GOC:TermGenie Definition: Any process that activates or increases the frequency, rate or extent of camalexin biosynthetic process.